{
  "gene": "UniProtKB:P0DOY5",
  "term_label": "Unknown molecular function",
  "term_id": "UNKNOWN:0001",
  "gene_name": "Immunoglobulin heavy diversity 1-1",
  "gene_symbol": "IGHD1-1"
}